glutaryl-7-aminocephalosporanic-acid acylase activity [GO:0033968] (molecular function) Definition: Catalysis of the reaction: (7R)-7-(4-carboxybutanamido)cephalosporanate + H2O = (7R)-7-aminocephalosporanate + glutarate. Also known as: (7R)-7-(4-carboxybutanamido)cephalosporanate amidohydrolase activity, 7beta-(4-carboxybutanamido)cephalosporanic acid acylase activity, CA, GA, GCA, GL-7-ACA acylase activity, cephalosporin C acylase activity, cephalosporin acylase activity, glutaryl-7-ACA acylase activity, glutaryl-7-aminocephalosporanic acid acylase activity Sources: EC:3.5.1.93 Relationships: is a type of hydrolase activity, acting on carbon-nitrogen (but not peptide) bonds, in linear amides [GO:0016811]